{
  "term_id": "UNKNOWN:0003",
  "gene_name": "Headcase protein homolog",
  "term_label": "Unknown cellular component",
  "gene": "UniProtKB:Q9UBI9",
  "gene_symbol": "HECA"
}